regulation of apoptotic process involved in metanephric collecting duct development [GO:1900214] (biological process) References: PMID:17314325 Sources: GOC:TermGenie, GOC:mtg_kidney_jan10, GOC:yaf Definition: Any process that modulates the frequency, rate or extent of apoptotic process involved in metanephric collecting duct development. Subtypes: GO:1900215, positive regulation of apoptotic process involved in metanephric collecting duct development [GO:1900216] Relationships: is a type of regulation of apoptotic process involved in development [GO:1904748]; regulates GO:1900204 Also known as: regulation of apoptotic cell death of metanephric collecting duct development, regulation of apoptotic process of metanephric collecting duct development, regulation of apoptotic programmed cell death of metanephric collecting duct development, regulation of programmed cell death by apoptosis of metanephric collecting duct development, regulation of apoptosis of metanephric collecting duct development, regulation of apoptotic program of metanephric collecting duct development, regulation of type I programmed cell death of metanephric collecting duct development, regulation of signaling (initiator) caspase activity of metanephric collecting duct development